{
  "gene_symbol": "IRX6",
  "term_id": "GO:0006357",
  "gene": "UniProtKB:P78412",
  "term_label": "regulation of transcription by RNA polymerase II",
  "gene_name": "Iroquois-class homeodomain protein IRX-6"
}